{
  "term_id": "GO:0005737",
  "term_label": "cytoplasm",
  "gene_symbol": "GSTO1",
  "gene": "UniProtKB:P78417",
  "gene_name": "Glutathione S-transferase omega-1"
}